minus-end-directed vesicle transport along microtubule [GO:0072382] (biological process) Sources: GOC:BHF, GOC:mah Definition: The directed movement of a vesicle towards the minus end of a microtubule, mediated by motor proteins. This process begins with the attachment of a vesicle to a microtubule, and ends when the vesicle reaches its final destination. Also known as: microtubule minus-end-directed vesicle localization, microtubule minus-end-directed vesicle distribution Relationships: is a type of vesicle transport along microtubule [GO:0047496]; is a type of minus-end-directed organelle transport along microtubule [GO:0072385]